chondroitin sulfotransferase activity [GO:0034481] (MF) Sources: GOC:curators Subtypes: GO:0008459, chondroitin 2-sulfotransferase activity [GO:0034482], chondroitin 4-sulfotransferase activity [GO:0047756] Relationships: is a type of GO:0050698 Definition: Catalysis of the reaction: 3'-phosphoadenosine 5'-phosphosulfate + chondroitin = adenosine 3',5'-bisphosphate + chondroitin sulfate.